regulation of gamma-aminobutyric acid uptake involved in transmission of nerve impulse [GO:0051947] (biological process) Relationships: is a type of regulation of organic acid transport [GO:0032890]; is_a GO:0051941; regulates gamma-aminobutyric acid reuptake [GO:0051936] Subtypes: negative regulation of gamma-aminobutyric acid uptake involved in transmission of nerve impulse [GO:0051949], positive regulation of gamma-aminobutyric acid uptake involved in transmission of nerve impulse [GO:0051950] Sources: GOC:ai Also known as: regulation of 4-aminobutyrate reuptake, regulation of 4-aminobutyrate uptake during transmission of nerve impulse, regulation of GABA reuptake, regulation of GABA uptake during transmission of nerve impulse, regulation of gamma-aminobutyric acid reuptake, regulation of gamma-aminobutyric acid uptake involved in conduction of nerve impulse, regulation of gamma-aminobutyric acid uptake during transmission of nerve impulse Definition: Any process that modulates the frequency, rate or extent of the directed movement of gamma-aminobutyric acid (GABA, 4-aminobutyrate) into a neuron or glial cell.